regulation of corticotropin secretion [GO:0051459] (biological process) Subtypes: negative regulation of corticotropin secretion [GO:0051460], GO:0051461 Sources: GOC:ai, GOC:dph Relationships: is a type of GO:0044060; is a type of regulation of peptide hormone secretion [GO:0090276]; regulates corticotropin secretion [GO:0051458] Also known as: regulation of ACTH secretion, regulation of adrenocorticotropic hormone secretion, regulation of adrenocorticotropin secretion, regulation of adrenotropin hormone secretion, regulation of adrenotropin secretion, regulation of corticotropic hormone secretion Definition: Any process that modulates the frequency, rate or extent of the regulated release of corticotropic hormone from a cell.